{
  "gene_name": "Epidermal growth factor-like protein 7",
  "gene": "UniProtKB:Q9UHF1",
  "term_id": "GO:0005102",
  "gene_symbol": "EGFL7",
  "term_label": "signaling receptor binding"
}